glycoprotein Ib-IX-V complex [GO:1990779] (cellular component) Note: An example of this is GB1BA in human (P07359) in PMID:1730602 (inferred from direct assay). Definition: A transmembrane signaling receptor complex found exclusively on platelets. Involved in haemostasis and thrombosis where it aids blood coagulation. References: PMID:1730602, PMID:23336709, PMID:25297919 Sources: GOC:bhm Also known as: CD42, GPIb-IX-V complex, GPIb-V-IX complex Relationships: is a type of glycoprotein complex [GO:0090665]; is a type of plasma membrane signaling receptor complex [GO:0098802]